cellulose 1,4-beta-cellobiosidase activity (reducing end) [GO:0102252] (molecular function) Definition: Catalysis of the reaction: n H2O + a cellodextrin = n beta-cellobiose, releasing cellobiose from the reducing ends of the chains. Sources: EC:3.2.1.176, GOC:pz Relationships: is a type of hydrolase activity, hydrolyzing O-glycosyl compounds [GO:0004553]